{
  "term_id": "GO:0007155",
  "gene": "UniProtKB:O43930",
  "gene_symbol": "PRKY",
  "gene_name": "Putative serine_threonine-protein kinase PRKY",
  "term_label": "cell adhesion"
}